endogenous lipid antigen binding [GO:0030883] (molecular function) Relationships: is a type of lipid antigen binding [GO:0030882] Definition: Binding to an endogenous cellular lipid antigen. References: PMID:14500461